propylene metabolic process [GO:0018964] (biological process) Subtypes: propylene catabolic process [GO:0042208] Definition: The chemical reactions and pathways involving propylene, an alkene produced by catalytic or thermal cracking of hydrocarbons or as a by-product of petroleum refining. It is used mainly in the preparation of alkylates for gasoline and in the production of polypropylene, acrylonitrile, propylene oxide and a number of other industrial chemicals. Also known as: propylene metabolism Relationships: is a type of xenobiotic metabolic process [GO:0006805]; is a type of olefin metabolic process [GO:1900673] Sources: GOC:jl